{
  "gene_name": "Calcium-activated potassium channel subunit alpha-1",
  "gene": "UniProtKB:Q12791",
  "gene_symbol": "KCNMA1",
  "term_label": "vasodilation",
  "term_id": "GO:0042311"
}